cupric ion binding [GO:1903135] (molecular function) Relationships: is a type of copper ion binding [GO:0005507] References: PMID:24567322 Sources: GOC:PARL, GOC:TermGenie, GOC:bf, GO_REF:0000067 Also known as: Cu(2+) binding, Cu(II) binding, copper(2+)binding Definition: Binding to a cupric ion, copper(2+).